L-glutamate catabolic process via L-citramalate [GO:0019553] (biological process) Relationships: is a type of L-glutamate catabolic process [GO:0006538] Sources: GOC:go_curators Definition: The chemical reactions and pathways resulting in the breakdown of L-glutamate, via the intermediate L-citramalate. Also known as: glutamate breakdown via L-citramalate, glutamate degradation via L-citramalate